{
  "term_id": "GO:0005634",
  "term_label": "nucleus",
  "gene_name": "Ubiquitin-like modifier-activating enzyme 6",
  "gene_symbol": "UBA6",
  "gene": "UniProtKB:A0AVT1"
}